{
  "gene_name": "Neuronal acetylcholine receptor subunit alpha-6",
  "gene_symbol": "CHRNA6",
  "term_label": "neuron projection",
  "term_id": "GO:0043005",
  "gene": "UniProtKB:Q15825"
}